{
  "gene_name": "Mesothelin",
  "term_id": "UNKNOWN:0001",
  "gene_symbol": "MSLN",
  "term_label": "Unknown molecular function",
  "gene": "UniProtKB:Q13421"
}